chloroplast elongation [GO:0010151] (biological process) Definition: Expansion of the chloroplast that usually precedes division. Sources: GOC:lr Relationships: is a type of chloroplast organization [GO:0009658]